{
  "gene_symbol": "RUFY3",
  "term_label": "cytoplasm",
  "gene": "UniProtKB:Q7L099",
  "term_id": "GO:0005737",
  "gene_name": "Protein RUFY3"
}